1-alpha,25-dihydroxyvitamin D3 24-hydroxylase activity [GO:0030342] (molecular function) Relationships: is a type of vitamin D 24-hydroxylase activity [GO:0070576] References: PMID:8506296 Also known as: 1,25-(OH)2D3 24-hydroxylase activity, calcitriol 24-hydroxylase activity Definition: Catalysis of the hydroxylation of C-24 of 1-alpha,25-hydroxycholecalciferol (25-hydroxyvitamin D3; calcitriol).